{
  "term_id": "GO:0005783",
  "term_label": "endoplasmic reticulum",
  "gene_name": "Cell cycle control protein 50B",
  "gene_symbol": "TMEM30B",
  "gene": "UniProtKB:Q3MIR4"
}